{
  "gene_symbol": "MYPN",
  "term_id": "GO:0098632",
  "gene_name": "Myopalladin",
  "gene": "UniProtKB:Q86TC9",
  "term_label": "cell-cell adhesion mediator activity"
}